cellular response to biotin starvation [GO:1990383] (biological process) Definition: Any process that results in a change in state or activity of a cell (in terms of movement, secretion, enzyme production, gene expression, etc.) as a result of deprivation of biotin. References: PMID:12557275 Relationships: is_a cellular response to starvation [GO:0009267]